{
  "gene_symbol": "HOXC11",
  "gene_name": "Homeobox protein Hox-C11",
  "gene": "UniProtKB:O43248",
  "term_id": "GO:0000981",
  "term_label": "DNA-binding transcription factor activity, RNA polymerase II-specific"
}